double-stranded RNA binding [GO:0003725] (molecular function) Sources: GOC:jl Also known as: dsRNA binding Subtypes: RNA strand-exchange activity [GO:0034057], double-stranded miRNA binding [GO:0098851] Definition: Binding to double-stranded RNA. Relationships: is a type of GO:0003723